{
  "gene_name": "AT-rich interactive domain-containing protein 5A",
  "gene": "UniProtKB:Q03989",
  "gene_symbol": "ARID5A",
  "term_label": "transcription cis-regulatory region binding",
  "term_id": "GO:0000976"
}